{
  "gene_name": "General vesicular transport factor p115",
  "gene_symbol": "USO1",
  "gene": "UniProtKB:O60763",
  "term_id": "UNKNOWN:0001",
  "term_label": "Unknown molecular function"
}